{
  "gene_symbol": "DUSP18",
  "gene": "UniProtKB:Q8NEJ0",
  "gene_name": "Dual specificity protein phosphatase 18",
  "term_label": "protein tyrosine phosphatase activity",
  "term_id": "GO:0004725"
}